{
  "gene_symbol": "SLC38A5",
  "term_id": "GO:0015816",
  "gene": "UniProtKB:Q8WUX1",
  "gene_name": "Sodium-coupled neutral amino acid transporter 5",
  "term_label": "glycine transport"
}